{
  "gene_name": "Tyrosine-protein phosphatase non-receptor type 13",
  "gene": "UniProtKB:Q12923",
  "term_id": "GO:0004725",
  "gene_symbol": "PTPN13",
  "term_label": "protein tyrosine phosphatase activity"
}